{
  "gene": "UniProtKB:Q5T200",
  "gene_symbol": "ZC3H13",
  "term_label": "Unknown biological process",
  "gene_name": "Zinc finger CCCH domain-containing protein 13",
  "term_id": "UNKNOWN:0002"
}